D-mannose binding [GO:0005537] (molecular function) Relationships: is a type of GO:0048029 Sources: GOC:jl, ISBN:0192800981 Also known as: mannose binding, mannose binding lectin Definition: Binding to mannose, a monosaccharide hexose, stereoisomeric with glucose, that occurs naturally only in polymerized forms called mannans.